{
  "gene": "UniProtKB:Q50LG9",
  "term_label": "positive regulation of synapse assembly",
  "gene_name": "Leucine-rich repeat-containing protein 24",
  "gene_symbol": "LRRC24",
  "term_id": "GO:0051965"
}